{
  "gene_symbol": "CRACDL",
  "term_label": "Unknown biological process",
  "gene_name": "CRACD-like protein",
  "term_id": "UNKNOWN:0002",
  "gene": "UniProtKB:Q6NV74"
}